{
  "gene": "UniProtKB:Q5SXH7",
  "term_id": "UNKNOWN:0002",
  "term_label": "Unknown biological process",
  "gene_symbol": "PLEKHS1",
  "gene_name": "Pleckstrin homology domain-containing family S member 1"
}